{
  "gene_symbol": "IPMK",
  "term_label": "nucleus",
  "gene": "UniProtKB:Q8NFU5",
  "term_id": "GO:0005634",
  "gene_name": "Inositol polyphosphate multikinase"
}